{
  "gene_symbol": "NELFE",
  "term_id": "GO:0032021",
  "term_label": "NELF complex",
  "gene": "UniProtKB:P18615",
  "gene_name": "Negative elongation factor E"
}